{
  "term_id": "GO:0003743",
  "gene": "UniProtKB:P20042",
  "gene_symbol": "EIF2S2",
  "term_label": "translation initiation factor activity",
  "gene_name": "Eukaryotic translation initiation factor 2 subunit 2"
}